{
  "gene_name": "Tumor necrosis factor ligand superfamily member 11",
  "term_id": "GO:0007166",
  "gene_symbol": "TNFSF11",
  "gene": "UniProtKB:O14788",
  "term_label": "cell surface receptor signaling pathway"
}